{
  "gene": "UniProtKB:Q9HCS2",
  "gene_name": "Cytochrome P450 4F12",
  "term_id": "GO:0042376",
  "gene_symbol": "CYP4F12",
  "term_label": "phylloquinone catabolic process"
}